{
  "term_label": "membrane",
  "gene_name": "Solute carrier family 15 member 5",
  "gene_symbol": "SLC15A5",
  "gene": "UniProtKB:A6NIM6",
  "term_id": "GO:0016020"
}